{
  "gene": "UniProtKB:P08238",
  "gene_symbol": "HSP90AB1",
  "term_id": "GO:0005829",
  "gene_name": "Heat shock protein HSP 90-beta",
  "term_label": "cytosol"
}